NAD+ kinase activity [GO:0003951] (molecular function) Relationships: is a type of kinase activity [GO:0016301]; is a type of phosphotransferase activity, alcohol group as acceptor [GO:0016773] Also known as: NAD kinase activity, ATP:NAD+ 2'-phosphotransferase activity, DPN kinase activity, NADK, nicotinamide adenine dinucleotide kinase (phosphorylating), nicotinamide adenine dinucleotide kinase activity Sources: RHEA:18629 Definition: Catalysis of the reaction: ATP + NAD+ = ADP + H+ + NADP+.